peripheral nervous system myelin formation [GO:0032290] (biological process) Also known as: myelin formation in peripheral nervous system, peripheral nervous system myelin sheath formation Relationships: is a type of myelin assembly [GO:0032288]; is part of GO:0022011 Definition: The process in which the wraps of cell membrane that constitute myelin are laid down around an axon by Schwann cells in the peripheral nervous system. Sources: GOC:dgh